chondrocyte differentiation [GO:0002062] (biological process) Definition: The process in which a chondroblast acquires specialized structural and/or functional features of a chondrocyte. A chondrocyte is a polymorphic cell that forms cartilage. Sources: GOC:dph Relationships: is a type of GO:0030154; is part of GO:0051216 Subtypes: chondrocyte differentiation involved in endochondral bone morphogenesis [GO:0003413] Regulation: regulated by regulation of chondrocyte differentiation [GO:0032330]; negatively regulated by negative regulation of chondrocyte differentiation [GO:0032331]; positively regulated by positive regulation of chondrocyte differentiation [GO:0032332]